{
  "term_id": "GO:0070830",
  "gene": "UniProtKB:Q9BTW9",
  "term_label": "bicellular tight junction assembly",
  "gene_name": "Tubulin-specific chaperone D",
  "gene_symbol": "TBCD"
}